{
  "gene_symbol": "FEM1B",
  "term_label": "nucleus",
  "gene": "UniProtKB:Q9UK73",
  "term_id": "GO:0005634",
  "gene_name": "Protein fem-1 homolog B"
}